{
  "gene_symbol": "GTF2B",
  "gene": "UniProtKB:Q00403",
  "term_id": "GO:0006352",
  "term_label": "DNA-templated transcription initiation",
  "gene_name": "Transcription initiation factor IIB"
}